{
  "gene_name": "Testis-specific Y-encoded-like protein 4",
  "term_label": "chromatin binding",
  "gene_symbol": "TSPYL4",
  "term_id": "GO:0003682",
  "gene": "UniProtKB:Q9UJ04"
}